positive regulation of R7 cell differentiation [GO:0045678] (biological process) Relationships: is a type of regulation of R7 cell differentiation [GO:0045676]; is a type of positive regulation of compound eye photoreceptor cell differentiation [GO:0110117]; positively regulates R7 cell differentiation [GO:0045466] Also known as: positive regulation of R7 differentiation, up regulation of R7 differentiation, up-regulation of R7 differentiation, upregulation of R7 differentiation, activation of R7 differentiation, stimulation of R7 differentiation Sources: GOC:dph, GOC:go_curators, GOC:tb Definition: Any process that activates or increases the frequency, rate or extent of R7 cell differentiation.